{
  "term_label": "negative regulation of G2/M transition of mitotic cell cycle",
  "term_id": "GO:0010972",
  "gene": "UniProtKB:Q9NQS1",
  "gene_name": "Cell death regulator Aven",
  "gene_symbol": "AVEN"
}